{
  "gene": "UniProtKB:P35268",
  "gene_symbol": "RPL22",
  "gene_name": "Large ribosomal subunit protein eL22",
  "term_label": "structural constituent of ribosome",
  "term_id": "GO:0003735"
}